glial cell migration in anterior lateral line nerve [GO:0048912] (biological process) Relationships: is a type of lateral line nerve glial cell migration [GO:0048896]; BFO_0000050 anterior lateral line nerve development [GO:0048909] Definition: The movement of a glial cell along the axons in the anterior lateral line nerve. References: PMID:12062041